{
  "gene_name": "Microtubule-associated protein 4",
  "gene_symbol": "MAP4",
  "term_label": "neuron projection",
  "gene": "UniProtKB:P27816",
  "term_id": "GO:0043005"
}